{
  "term_label": "GABA-A receptor activity",
  "gene_symbol": "GABRR1",
  "term_id": "GO:0004890",
  "gene_name": "Gamma-aminobutyric acid receptor subunit rho-1",
  "gene": "UniProtKB:P24046"
}